negative regulation of fusion of virus membrane with host plasma membrane [GO:1903914] (BP) Also known as: down regulation of fusion of virus membrane with host plasma membrane, down regulation of viral envelope fusion with host cell membrane, down regulation of viral envelope fusion with host membrane, down regulation of viral envelope fusion with host plasma membrane, down regulation of viral penetration via membrane fusion, down-regulation of fusion of virus membrane with host plasma membrane, down-regulation of viral envelope fusion with host cell membrane, down-regulation of viral envelope fusion with host membrane, down-regulation of viral envelope fusion with host plasma membrane, down-regulation of viral penetration via membrane fusion, downregulation of fusion of virus membrane with host plasma membrane, downregulation of viral envelope fusion with host cell membrane, downregulation of viral envelope fusion with host membrane, downregulation of viral envelope fusion with host plasma membrane, downregulation of viral penetration via membrane fusion, negative regulation of viral envelope fusion with host cell membrane, negative regulation of viral envelope fusion with host membrane, negative regulation of viral envelope fusion with host plasma membrane, negative regulation of viral penetration via membrane fusion, inhibition of fusion of virus membrane with host plasma membrane, inhibition of viral envelope fusion with host cell membrane, inhibition of viral envelope fusion with host membrane, inhibition of viral envelope fusion with host plasma membrane, inhibition of viral penetration via membrane fusion, down regulation of viral entry into host cell via membrane fusion with the plasma membrane, down regulation of viral-cell fusion molecule activity, down-regulation of viral entry into host cell via membrane fusion with the plasma membrane, down-regulation of viral-cell fusion molecule activity, downregulation of viral entry into host cell via membrane fusion with the plasma membrane, downregulation of viral-cell fusion molecule activity, inhibition of viral entry into host cell via membrane fusion with the plasma membrane, inhibition of viral-cell fusion molecule activity, negative regulation of viral entry into host cell via membrane fusion with the plasma membrane, negative regulation of viral-cell fusion molecule activity Definition: Any process that stops, prevents or reduces the frequency, rate or extent of fusion of virus membrane with host plasma membrane. Relationships: is a type of negative regulation of viral process [GO:0048525]; is a type of negative regulation of cellular component organization [GO:0051129]; is a type of regulation of fusion of virus membrane with host plasma membrane [GO:1903913]; negatively regulates fusion of virus membrane with host plasma membrane [GO:0019064]; negatively regulates symbiont entry into host cell [GO:0046718] References: PMID:23575248 Sources: GOC:TermGenie, GOC:als, GO_REF:0000058